positive regulation of sporulation [GO:0043938] (biological process) Sources: GOC:pamgo_curators Definition: Any process that activates, maintains or increases the frequency, rate or extent of sporulation, the process whose specific outcome is the progression of a spore over time, from its initiation to the mature structure. Relationships: is a type of regulation of sporulation [GO:0043937]; is a type of GO:0051094; positively regulates sporulation [GO:0043934] Subtypes: positive regulation of sporulation resulting in formation of a cellular spore [GO:0045881], positive regulation of conidium formation [GO:0075307], positive regulation of oomycete sporangium development [GO:0075323]